{
  "gene": "UniProtKB:Q9Y3I1",
  "gene_symbol": "FBXO7",
  "gene_name": "F-box only protein 7",
  "term_label": "positive regulation of autophagy of mitochondrion",
  "term_id": "GO:1903599"
}